{
  "gene_symbol": "UGT1A10",
  "term_label": "UDP-glycosyltransferase activity",
  "gene": "UniProtKB:Q9HAW8",
  "gene_name": "UDP-glucuronosyltransferase 1A10",
  "term_id": "GO:0008194"
}